regulation of sodium ion export across plasma membrane [GO:1903276] (biological process) Subtypes: negative regulation of sodium ion export across plasma membrane [GO:1903277], positive regulation of sodium ion export across plasma membrane [GO:1903278] Also known as: regulation of sodium ion export from cell, regulation of sodium export, regulation of sodium ion export Definition: Any process that modulates the frequency, rate or extent of sodium ion export across the plasma membrane. Relationships: is a type of regulation of sodium ion transmembrane transport [GO:1902305]; regulates sodium ion export across plasma membrane [GO:0036376] References: PMID:17095720 Sources: GOC:BHF, GOC:TermGenie, GOC:rl, GO_REF:0000058